{
  "gene": "UniProtKB:P04439",
  "gene_name": "HLA class I histocompatibility antigen, A alpha chain",
  "term_id": "GO:0030881",
  "gene_symbol": "HLA-A",
  "term_label": "beta-2-microglobulin binding"
}